{
  "term_label": "CDP-diacylglycerol biosynthetic process",
  "term_id": "GO:0016024",
  "gene_symbol": "CDS2",
  "gene": "UniProtKB:O95674",
  "gene_name": "Phosphatidate cytidylyltransferase 2"
}